histamine biosynthetic process [GO:0001694] (biological process) Definition: The chemical reactions and pathways resulting in the formation of histamine, a physiologically active amine, found in plant and animal tissue and released from mast cells as part of an allergic reaction in humans. Relationships: is a type of GO:0001692; is a type of biogenic amine biosynthetic process [GO:0042401] Also known as: histamine anabolism, histamine biosynthesis, histamine formation, histamine synthesis Sources: GOC:jl, ISBN:0395825172